rhamnose biosynthetic process [GO:0019300] (biological process) Definition: The chemical reactions and pathways resulting in the formation of rhamnose, the hexose 6-deoxy-L-mannose. Also known as: rhamnose anabolism, rhamnose biosynthesis, rhamnose formation, rhamnose synthesis Sources: ISBN:0198506732 Relationships: is a type of hexose biosynthetic process [GO:0019319]